{
  "gene": "UniProtKB:Q9NZH6",
  "gene_symbol": "IL37",
  "gene_name": "Interleukin-37",
  "term_id": "GO:0005654",
  "term_label": "nucleoplasm"
}